{
  "term_label": "Unknown cellular component",
  "gene_symbol": "CCDC171",
  "term_id": "UNKNOWN:0003",
  "gene_name": "Coiled-coil domain-containing protein 171",
  "gene": "UniProtKB:Q6TFL3"
}